{
  "term_label": "Unknown biological process",
  "gene_name": "Olfactory receptor 51I1",
  "gene": "UniProtKB:Q9H343",
  "term_id": "UNKNOWN:0002",
  "gene_symbol": "OR51I1"
}